{
  "gene_name": "Copine-9",
  "term_id": "GO:0005544",
  "gene_symbol": "CPNE9",
  "term_label": "calcium-dependent phospholipid binding",
  "gene": "UniProtKB:Q8IYJ1"
}